{
  "gene": "UniProtKB:P02746",
  "term_label": "Unknown cellular component",
  "term_id": "UNKNOWN:0003",
  "gene_symbol": "C1QB",
  "gene_name": "Complement C1q subcomponent subunit B"
}